{
  "gene_name": "1-acyl-sn-glycerol-3-phosphate acyltransferase alpha",
  "term_id": "GO:0006654",
  "term_label": "phosphatidic acid biosynthetic process",
  "gene_symbol": "AGPAT1",
  "gene": "UniProtKB:Q99943"
}